{
  "gene_name": "GPI-anchor transamidase",
  "term_id": "GO:0016255",
  "gene_symbol": "PIGK",
  "term_label": "attachment of GPI anchor to protein",
  "gene": "UniProtKB:Q92643"
}